{
  "gene_name": "Brain-derived neurotrophic factor",
  "term_id": "GO:0007169",
  "gene_symbol": "BDNF",
  "gene": "UniProtKB:P23560",
  "term_label": "cell surface receptor protein tyrosine kinase signaling pathway"
}